{
  "gene": "UniProtKB:Q9Y5Z0",
  "gene_symbol": "BACE2",
  "gene_name": "Beta-secretase 2",
  "term_label": "protein processing",
  "term_id": "GO:0016485"
}